{
  "gene": "UniProtKB:A0A0B4J2H0",
  "term_label": "Unknown cellular component",
  "term_id": "UNKNOWN:0003",
  "gene_name": "Immunoglobulin heavy variable 1-69D",
  "gene_symbol": "IGHV1-69D"
}